embryonic placenta morphogenesis [GO:0060669] (biological process) Definition: The process in which the embryonic placenta is generated and organized. Relationships: is a type of embryonic morphogenesis [GO:0048598]; is part of GO:0001892 Sources: GOC:dph